vitamin B6 transmembrane transporter activity [GO:0031924] (molecular function) Relationships: is_a GO:0090482; is part of vitamin B6 transport [GO:0031919] Definition: Enables the transfer of any of the vitamin B6 compounds, pyridoxal, pyridoxamine and pyridoxine and the active form, pyridoxal phosphate, from one side of a membrane to the other. Also known as: vitamin B6 transporter activity Sources: GOC:mah